ergothioneine biosynthesis from histidine via hercynylcysteine sulfoxide synthase [GO:0140479] (biological process) References: PMID:22209968, PMID:24828577 Relationships: is a type of ergothioneine biosynthetic process [GO:0052699] Definition: A biosynthetic process that results in the formation of ergothioneine from histidine via a set of steps including the hercynylcysteine sulfoxide synthase reaction, which converts N-alpha,N-alpha,N-alpha-trimethyl-L-histidine directly to hercynylcysteine sulfoxide.